{
  "gene": "UniProtKB:P20382",
  "term_label": "Unknown cellular component",
  "term_id": "UNKNOWN:0003",
  "gene_symbol": "PMCH",
  "gene_name": "Pro-MCH"
}